{
  "gene_symbol": "KCNQ2",
  "gene_name": "Potassium voltage-gated channel subfamily KQT member 2",
  "term_label": "voltage-gated potassium channel activity",
  "term_id": "GO:0005249",
  "gene": "UniProtKB:O43526"
}